{
  "term_label": "mRNA splice site recognition",
  "term_id": "GO:0006376",
  "gene_symbol": "LUC7L3",
  "gene": "UniProtKB:O95232",
  "gene_name": "Luc7-like protein 3"
}